antigen processing and presentation of exogenous antigen [GO:0019884] (biological process) References: PMID:15771591, PMID:15928678 Sources: GOC:add, ISBN:0781735149 Subtypes: antigen processing and presentation of exogenous peptide antigen [GO:0002478], antigen processing and presentation, exogenous lipid antigen via MHC class Ib [GO:0048007] Relationships: is a type of antigen processing and presentation [GO:0019882] Also known as: antigen presentation, exogenous antigen Definition: The process in which an antigen-presenting cell expresses antigen (peptide or lipid) of exogenous origin on its cell surface in association with an MHC protein complex.